modulation of symbiont haustorium neck formation for entry into host [GO:0075198] (biological process) Note: Note that this term should not be used to annotate gene products of the host. It should only be used to annotate those gene products from the symbiont involved in this process. Sources: GOC:pamgo_curators Definition: Any process that modulates the frequency, rate or extent of symbiont haustorium neck formation for entry into host. The host is defined as the larger of the organisms involved in a symbiotic interaction. Relationships: is a type of modulation of formation of structure involved in a symbiotic process [GO:0044145]; is a type of GO:0050793; is a type of modulation by symbiont of entry into host [GO:0052372]; regulates haustorium neck formation [GO:0075197] Subtypes: positive regulation of symbiont haustorium neck formation for entry into host [GO:0075199]